{
  "gene": "UniProtKB:Q8N4V1",
  "term_label": "early endosome",
  "gene_name": "ER membrane protein complex subunit 5",
  "gene_symbol": "MMGT1",
  "term_id": "GO:0005769"
}